{
  "term_label": "negative regulation of retrograde protein transport, ER to cytosol",
  "gene": "UniProtKB:Q8NHG7",
  "term_id": "GO:1904153",
  "gene_symbol": "SVIP",
  "gene_name": "Small VCP_p97-interacting protein"
}